pterocarpan synthase activity [GO:0140859] (molecular function) References: PMID:7805842 Sources: RHEA:35407 Definition: Catalysis of the reaction: H2O + medicarpin = 4'-methoxyisoflavan-2',4,7-triol. Also known as: 2',7-dihydroxy-4'-methoxyisoflavanol dehydratase activity, 2'-hydroxyisoflavanol 4,2'-dehydratase activity, 7,2'-dihydroxy-4'-methoxyisoflavanol dehydratase activity, medicarpan synthase activity, medicarpin synthase activity Relationships: is a type of hydro-lyase activity [GO:0016836]